{
  "gene_symbol": "TNNI3",
  "gene_name": "Troponin I, cardiac muscle",
  "term_id": "UNKNOWN:0001",
  "gene": "UniProtKB:P19429",
  "term_label": "Unknown molecular function"
}